{
  "gene": "UniProtKB:Q9C0F1",
  "gene_name": "Centrosomal protein of 44 kDa",
  "gene_symbol": "CEP44",
  "term_id": "GO:0007099",
  "term_label": "centriole replication"
}